methylitaconate delta-isomerase activity [GO:0050100] (molecular function) Sources: RHEA:23480 Definition: Catalysis of the reaction: 2-methylene-3-methylsuccinate = dimethylmaleate. Relationships: is a type of intramolecular oxidoreductase activity, transposing C=C bonds [GO:0016863] Also known as: methylitaconate D-isomerase activity, methylitaconate delta2-delta3-isomerase activity, methylitaconate isomerase activity